{
  "gene": "UniProtKB:Q7L7V1",
  "gene_name": "Putative pre-mRNA-splicing factor ATP-dependent RNA helicase DHX32",
  "term_id": "GO:0003723",
  "term_label": "RNA binding",
  "gene_symbol": "DHX32"
}